{
  "gene_name": "Heat shock factor-binding protein 1",
  "term_id": "GO:0005829",
  "gene": "UniProtKB:O75506",
  "gene_symbol": "HSBP1",
  "term_label": "cytosol"
}